{
  "term_label": "Rad6-Rad18 complex",
  "gene": "UniProtKB:Q9NS91",
  "term_id": "GO:0097505",
  "gene_symbol": "RAD18",
  "gene_name": "E3 ubiquitin-protein ligase RAD18"
}